{
  "gene": "UniProtKB:Q4G0S4",
  "term_id": "GO:1904768",
  "gene_symbol": "CYP27C1",
  "gene_name": "Cytochrome P450 27C1",
  "term_label": "all-trans-retinol binding"
}